mRNA (adenine-N1-)-methyltransferase activity [GO:0061953] (molecular function) References: PMID:29072297 Relationships: is a type of GO:0008174 Definition: Catalysis of the reaction: S-adenosyl-L-methionine + adenine in mRNA = S-adenosyl-L-homocysteine + N(1)-methyladenine in mRNA.